{
  "term_id": "GO:0061630",
  "term_label": "ubiquitin protein ligase activity",
  "gene_name": "E3 ubiquitin-protein ligase UHRF1",
  "gene": "UniProtKB:Q96T88",
  "gene_symbol": "UHRF1"
}